{
  "term_id": "GO:0005634",
  "gene_symbol": "ESRRA",
  "gene_name": "Steroid hormone receptor ERR1",
  "term_label": "nucleus",
  "gene": "UniProtKB:P11474"
}